{
  "gene_name": "Ataxin-3",
  "term_id": "GO:0006515",
  "gene_symbol": "ATXN3",
  "term_label": "protein quality control for misfolded or incompletely synthesized proteins",
  "gene": "UniProtKB:P54252"
}